amylopectin binding [GO:2001066] (molecular function) Sources: GOC:mengo_curators Definition: Binding to amylopectin. Relationships: is a type of carbohydrate derivative binding [GO:0097367]